regulation of beta-lactamase activity [GO:0033252] (biological process) Definition: Any process that modulates the frequency, rate or extent of beta-lactamase activity, the hydrolysis of a beta-lactam to yield a substituted beta-amino acid. Relationships: is a type of regulation of hydrolase activity [GO:0051336]; regulates beta-lactamase activity [GO:0008800] Sources: GOC:mah